{
  "gene_name": "Protein ZAR1-like",
  "term_label": "mRNA 3'-UTR binding",
  "gene_symbol": "ZAR1L",
  "term_id": "GO:0003730",
  "gene": "UniProtKB:A6NP61"
}